{
  "gene": "UniProtKB:Q92841",
  "gene_name": "Probable ATP-dependent RNA helicase DDX17",
  "term_id": "GO:0003729",
  "term_label": "mRNA binding",
  "gene_symbol": "DDX17"
}